{
  "term_label": "Unknown biological process",
  "term_id": "UNKNOWN:0002",
  "gene_symbol": "RLN1",
  "gene_name": "Prorelaxin H1",
  "gene": "UniProtKB:P04808"
}